{
  "term_label": "cytoplasm",
  "gene_name": "Protein HEXIM1",
  "gene": "UniProtKB:O94992",
  "gene_symbol": "HEXIM1",
  "term_id": "GO:0005737"
}